{
  "term_id": "GO:0000978",
  "term_label": "RNA polymerase II cis-regulatory region sequence-specific DNA binding",
  "gene_symbol": "KLF17",
  "gene": "UniProtKB:Q5JT82",
  "gene_name": "Krueppel-like factor 17"
}